{
  "term_label": "Unknown biological process",
  "gene_symbol": "OTUD6A",
  "gene": "UniProtKB:Q7L8S5",
  "term_id": "UNKNOWN:0002",
  "gene_name": "OTU domain-containing protein 6A"
}